{
  "gene": "UniProtKB:A0A096LPK9",
  "term_id": "UNKNOWN:0002",
  "term_label": "Unknown biological process",
  "gene_symbol": "OR4N4C",
  "gene_name": "Olfactory receptor 4N4C"
}